{
  "gene_symbol": "RAX",
  "term_id": "UNKNOWN:0003",
  "term_label": "Unknown cellular component",
  "gene_name": "Retinal homeobox protein Rx",
  "gene": "UniProtKB:Q9Y2V3"
}